{
  "gene": "UniProtKB:Q9UJ42",
  "gene_symbol": "GPR160",
  "term_id": "UNKNOWN:0001",
  "term_label": "Unknown molecular function",
  "gene_name": "Probable G-protein coupled receptor 160"
}